{
  "term_label": "mitochondrial outer membrane translocase complex",
  "gene_symbol": "TOMM5",
  "term_id": "GO:0005742",
  "gene_name": "Mitochondrial import receptor subunit TOM5 homolog",
  "gene": "UniProtKB:Q8N4H5"
}